{
  "gene": "UniProtKB:P35240",
  "gene_name": "Merlin",
  "term_id": "GO:0030175",
  "term_label": "filopodium",
  "gene_symbol": "NF2"
}